{
  "term_label": "extracellular space",
  "gene_name": "Interferon alpha-2",
  "term_id": "GO:0005615",
  "gene_symbol": "IFNA2",
  "gene": "UniProtKB:P01563"
}